{
  "gene_name": "Four and a half LIM domains protein 2",
  "gene_symbol": "FHL2",
  "term_label": "transcription corepressor activity",
  "gene": "UniProtKB:Q14192",
  "term_id": "GO:0003714"
}